{
  "gene": "UniProtKB:Q13496",
  "gene_symbol": "MTM1",
  "gene_name": "Myotubularin",
  "term_label": "cytoplasm",
  "term_id": "GO:0005737"
}